{
  "term_id": "GO:0042393",
  "gene": "UniProtKB:O60885",
  "gene_symbol": "BRD4",
  "term_label": "histone binding",
  "gene_name": "Bromodomain-containing protein 4"
}